{
  "gene_symbol": "ZSWIM5",
  "gene_name": "Zinc finger SWIM domain-containing protein 5",
  "term_label": "Unknown molecular function",
  "gene": "UniProtKB:Q9P217",
  "term_id": "UNKNOWN:0001"
}